{
  "term_label": "endoplasmic reticulum membrane",
  "term_id": "GO:0005789",
  "gene_symbol": "RETREG1",
  "gene": "UniProtKB:Q9H6L5",
  "gene_name": "Reticulophagy regulator 1"
}